{
  "gene_name": "Tumor necrosis factor ligand superfamily member 4",
  "term_id": "GO:0005615",
  "term_label": "extracellular space",
  "gene": "UniProtKB:P23510",
  "gene_symbol": "TNFSF4"
}